mesonephric distal tubule morphogenesis [GO:0061273] (biological process) Relationships: is a type of mesonephric nephron tubule morphogenesis [GO:0061240]; is a type of distal tubule morphogenesis [GO:0072156]; is part of mesonephric distal tubule development [GO:0061274] Definition: The process in which the anatomical structures of a mesonephric distal tubule are generated and organized. The mesonephric distal tubule is a mesonephric nephron tubule that begins at the macula densa and extends to the mesonephric connecting tubule. Sources: GOC:mtg_kidney_jan10